{
  "term_label": "protein K63-linked ubiquitination",
  "gene": "UniProtKB:Q15819",
  "gene_symbol": "UBE2V2",
  "term_id": "GO:0070534",
  "gene_name": "Ubiquitin-conjugating enzyme E2 variant 2"
}